{
  "term_id": "GO:0030672",
  "gene_symbol": "STX12",
  "gene_name": "Syntaxin-12",
  "gene": "UniProtKB:Q86Y82",
  "term_label": "synaptic vesicle membrane"
}